{
  "gene": "UniProtKB:P19087",
  "gene_symbol": "GNAT2",
  "term_id": "GO:0001750",
  "gene_name": "Guanine nucleotide-binding protein G(t) subunit alpha-2",
  "term_label": "photoreceptor outer segment"
}